pattern recognition receptor signaling pathway [GO:0002221] (biological process) Regulation: regulated by regulation of pattern recognition receptor signaling pathway [GO:0062207]; positively regulated by positive regulation of pattern recognition receptor signaling pathway [GO:0062208] Definition: The series of molecular signals initiated by a ligand binding to a pattern recognition receptor (PRR), and ending with the regulation of a downstream cellular process, e.g. transcription. PRRs bind pathogen-associated molecular pattern (PAMPs), structures conserved among microbial species, or damage-associated molecular pattern (DAMPs), endogenous molecules released from damaged cells. Relationships: is a type of innate immune response-activating signaling pathway [GO:0002758] References: PMID:15199967 Sources: GOC:add, GOC:ar, ISBN:0781735149 Also known as: PRR signaling pathway, pathogen receptor signaling pathway, pathogen receptor signalling pathway Subtypes: toll-like receptor signaling pathway [GO:0002224], cell surface pattern recognition receptor signaling pathway [GO:0002752], GO:0002753, peptidoglycan recognition protein signaling pathway [GO:0061057], pathogen-associated molecular pattern receptor signaling pathway [GO:0140426]